{
  "term_label": "Unknown molecular function",
  "gene": "UniProtKB:Q8N4B4",
  "term_id": "UNKNOWN:0001",
  "gene_name": "F-box only protein 39",
  "gene_symbol": "FBXO39"
}